{
  "term_label": "Unknown cellular component",
  "gene_symbol": "SAPCD1",
  "gene": "UniProtKB:Q5SSQ6",
  "term_id": "UNKNOWN:0003",
  "gene_name": "Suppressor APC domain-containing protein 1"
}